response to carbohydrate [GO:0009743] (biological process) Subtypes: detection of carbohydrate stimulus [GO:0009730], response to mannitol [GO:0010555], response to monosaccharide [GO:0034284], response to disaccharide [GO:0034285], response to pullulan [GO:0044592], defense response by callose deposition [GO:0052542], GO:0071322, response to sorbitol [GO:0072708], response to raffinose [GO:1901545] Relationships: is a type of response to oxygen-containing compound [GO:1901700] Definition: Any process that results in a change in state or activity of a cell or an organism (in terms of movement, secretion, enzyme production, gene expression, etc.) as a result of a carbohydrate stimulus. Also known as: response to carbohydrate stimulus Sources: GOC:jl